{
  "gene_symbol": "OR2C3",
  "term_label": "plasma membrane",
  "gene_name": "Olfactory receptor 2C3",
  "gene": "UniProtKB:Q8N628",
  "term_id": "GO:0005886"
}